{
  "gene": "UniProtKB:Q13459",
  "term_label": "lamellipodium morphogenesis",
  "gene_symbol": "MYO9B",
  "term_id": "GO:0072673",
  "gene_name": "Unconventional myosin-IXb"
}